{
  "term_label": "Unknown cellular component",
  "gene_name": "Late cornified envelope protein 2A",
  "gene": "UniProtKB:Q5TA79",
  "gene_symbol": "LCE2A",
  "term_id": "UNKNOWN:0003"
}